{
  "gene_name": "Uncharacterized protein",
  "gene_symbol": "A0A8V8TLL3",
  "term_id": "UNKNOWN:0003",
  "gene": "UniProtKB:A0A8V8TLL3",
  "term_label": "Unknown cellular component"
}